{
  "gene_name": "Uncharacterized protein CLBA1",
  "term_id": "GO:0032588",
  "gene": "UniProtKB:Q96F83",
  "gene_symbol": "CLBA1",
  "term_label": "trans-Golgi network membrane"
}